axon arborization [GO:0140060] (biological process) Definition: The process in which the terminal anatomical structures of an axon are generated and organized into branches of specialised projections, or boutons. An axon is the long process of a neuron that conducts nerve impulses, usually away from the cell body to the terminal branches. Relationships: is_a axonogenesis [GO:0007409]; is a type of neuron projection arborization [GO:0140058] References: PMID:23764288 Sources: GOC:aruk, GOC:bc